{
  "gene_name": "Taste receptor type 2 member 30",
  "gene": "UniProtKB:P59541",
  "gene_symbol": "TAS2R30",
  "term_id": "GO:0001580",
  "term_label": "detection of chemical stimulus involved in sensory perception of bitter taste"
}